{
  "term_label": "cell-cell signaling",
  "gene_symbol": "GJA8",
  "gene_name": "Gap junction alpha-8 protein",
  "term_id": "GO:0007267",
  "gene": "UniProtKB:P48165"
}